{
  "term_id": "GO:0005783",
  "term_label": "endoplasmic reticulum",
  "gene_name": "PAT complex subunit CCDC47",
  "gene": "UniProtKB:Q96A33",
  "gene_symbol": "CCDC47"
}